{
  "gene": "UniProtKB:P08571",
  "gene_name": "Monocyte differentiation antigen CD14",
  "term_label": "cellular response to lipopolysaccharide",
  "term_id": "GO:0071222",
  "gene_symbol": "CD14"
}